{
  "gene": "UniProtKB:Q9NNW5",
  "term_label": "tRNA methylation",
  "term_id": "GO:0030488",
  "gene_name": "WD repeat-containing protein 6",
  "gene_symbol": "WDR6"
}